{
  "gene": "UniProtKB:Q6ZT21",
  "gene_symbol": "TMPPE",
  "gene_name": "Transmembrane protein with metallophosphoesterase domain",
  "term_id": "UNKNOWN:0002",
  "term_label": "Unknown biological process"
}